gastrulation involving germ band extension [GO:0010004] (biological process) Sources: GOC:go_curators, GOC:mtg_sensu Relationships: is a type of gastrulation with mouth forming first [GO:0001703] Definition: A complex and coordinated series of cellular movements, including germ band extension, that occurs at the end of cleavage during embryonic development. An example of this process is found in Drosophila melanogaster.